retrograde extension [GO:0003389] (biological process) Subtypes: dendrite development by retrograde extension [GO:0003390] Sources: GOC:ascb_2009, GOC:dph, GOC:tb Relationships: is a type of neuron projection development [GO:0031175] Definition: The progression of a neuronal projection over time by the attachment of a part of the cell to an anchor and the subsequent migration of the cell body away from the anchor point.